{
  "term_id": "GO:0043291",
  "gene_name": "DmX-like protein 2",
  "gene_symbol": "DMXL2",
  "gene": "UniProtKB:Q8TDJ6",
  "term_label": "RAVE complex"
}